{
  "gene_symbol": "OCR1",
  "gene_name": "Ovarian cancer-related protein 1",
  "term_label": "Unknown molecular function",
  "gene": "UniProtKB:Q9BZK8",
  "term_id": "UNKNOWN:0001"
}